{
  "term_id": "GO:0000978",
  "gene_symbol": "ZNF324",
  "term_label": "RNA polymerase II cis-regulatory region sequence-specific DNA binding",
  "gene": "UniProtKB:O75467",
  "gene_name": "Zinc finger protein 324A"
}